{
  "gene_symbol": "PFDN1",
  "term_label": "protein folding chaperone",
  "gene": "UniProtKB:O60925",
  "gene_name": "Prefoldin subunit 1",
  "term_id": "GO:0044183"
}